{
  "gene": "UniProtKB:P22455",
  "term_id": "GO:0005886",
  "gene_symbol": "FGFR4",
  "term_label": "plasma membrane",
  "gene_name": "Fibroblast growth factor receptor 4"
}